{
  "term_label": "NMDA selective glutamate receptor complex",
  "gene_name": "Glutamate receptor ionotropic, NMDA 2D",
  "gene": "UniProtKB:O15399",
  "gene_symbol": "GRIN2D",
  "term_id": "GO:0017146"
}